cellular response to phosphate starvation [GO:0016036] (biological process) Sources: GOC:jl Regulation: positively regulated by GO:0080040; regulated by GO:0140255; negatively regulated by negative regulation of cellular response to phosphate starvation [GO:0140256] Relationships: is a type of cellular response to starvation [GO:0009267] Definition: Any process that results in a change in state or activity of a cell (in terms of movement, secretion, enzyme production, gene expression, etc.) as a result of deprivation of phosphate.